{
  "gene_symbol": "RNF152",
  "term_id": "GO:0010508",
  "gene": "UniProtKB:Q8N8N0",
  "term_label": "positive regulation of autophagy",
  "gene_name": "E3 ubiquitin-protein ligase RNF152"
}